{
  "gene_name": "Protein BEX3",
  "term_id": "GO:0005102",
  "gene_symbol": "BEX3",
  "term_label": "signaling receptor binding",
  "gene": "UniProtKB:Q00994"
}